germarium-derived egg chamber formation [GO:0007293] (biological process) Definition: Construction of a stage-1 egg chamber in the anterior part of the germarium, from the progeny of germ-line and somatic stem cells. An example of this is found in Drosophila melanogaster. Relationships: is a type of developmental process involved in reproduction [GO:0003006]; is_a GO:0048646; is part of oogenesis [GO:0048477] Sources: GOC:mtg_sensu, ISBN:0879694238